{
  "term_label": "nucleus",
  "gene_name": "Cytoplasmic polyadenylation element-binding protein 1",
  "term_id": "GO:0005634",
  "gene": "UniProtKB:Q9BZB8",
  "gene_symbol": "CPEB1"
}